{
  "term_id": "GO:0001530",
  "gene_name": "Bactericidal permeability-increasing protein",
  "term_label": "lipopolysaccharide binding",
  "gene": "UniProtKB:P17213",
  "gene_symbol": "BPI"
}